{
  "term_label": "establishment or maintenance of cell polarity regulating cell shape",
  "gene_symbol": "PARVB",
  "term_id": "GO:0071963",
  "gene": "UniProtKB:Q9HBI1",
  "gene_name": "Beta-parvin"
}